{
  "gene_name": "Serine protease 48",
  "gene": "UniProtKB:Q7RTY5",
  "term_id": "GO:0005615",
  "gene_symbol": "PRSS48",
  "term_label": "extracellular space"
}